{
  "gene_symbol": "ZNF514",
  "gene_name": "Zinc finger protein 514",
  "term_id": "GO:0000978",
  "gene": "UniProtKB:Q96K75",
  "term_label": "RNA polymerase II cis-regulatory region sequence-specific DNA binding"
}